L-cysteine catabolic process via cystine [GO:0019453] (biological process) Also known as: L-cysteine breakdown via cystine, L-cysteine degradation via cystine Relationships: is a type of L-cysteine catabolic process [GO:0019448] Sources: GOC:go_curators Subtypes: L-cysteine catabolic process via cystine, using glutathione-cystine transhydrogenase [GO:0019454], GO:0019455, L-cysteine catabolic process via cystine, using cysteine transaminase [GO:0019456] Definition: The chemical reactions and pathways resulting in the breakdown of L-cysteine, via the intermediate cystine.